{
  "gene_name": "Rap1 GTPase-activating protein 1",
  "term_id": "GO:0022407",
  "gene": "UniProtKB:P47736",
  "gene_symbol": "RAP1GAP",
  "term_label": "regulation of cell-cell adhesion"
}